{
  "term_label": "nucleus",
  "gene_symbol": "LPXN",
  "term_id": "GO:0005634",
  "gene": "UniProtKB:O60711",
  "gene_name": "Leupaxin"
}